{
  "gene_symbol": "CFAP53",
  "gene_name": "Cilia- and flagella-associated protein 53",
  "term_label": "Unknown cellular component",
  "gene": "UniProtKB:Q96M91",
  "term_id": "UNKNOWN:0003"
}